{
  "term_id": "GO:0000978",
  "gene_symbol": "ZNF275",
  "term_label": "RNA polymerase II cis-regulatory region sequence-specific DNA binding",
  "gene": "UniProtKB:Q9NSD4",
  "gene_name": "Zinc finger protein 275"
}